{
  "term_label": "cytoplasm",
  "term_id": "GO:0005737",
  "gene_symbol": "KIFC2",
  "gene": "UniProtKB:Q96AC6",
  "gene_name": "Kinesin-like protein KIFC2"
}